{
  "gene_symbol": "CCNT2",
  "gene_name": "Cyclin-T2",
  "gene": "UniProtKB:O60583",
  "term_label": "nucleus",
  "term_id": "GO:0005634"
}